{
  "gene_name": "tRNA (cytosine(38)-C(5))-methyltransferase",
  "term_label": "tRNA processing",
  "gene": "UniProtKB:O14717",
  "term_id": "GO:0008033",
  "gene_symbol": "TRDMT1"
}